rhamnulokinase activity [GO:0008993] (molecular function) Also known as: ATP:L-rhamnulose 1-phosphotransferase activity, L-rhamnulokinase activity, L-rhamnulose kinase activity, RhuK, rhamnulokinase (phosphorylating), rhamnulose kinase activity Sources: EC:2.7.1.5 Definition: Catalysis of the reaction: ATP + L-rhamnulose = ADP + L-rhamnulose 1-phosphate. Relationships: is_a GO:0016773; is a type of carbohydrate kinase activity [GO:0019200]